{
  "gene_symbol": "SUN5",
  "term_id": "GO:0034993",
  "gene_name": "SUN domain-containing protein 5",
  "gene": "UniProtKB:Q8TC36",
  "term_label": "meiotic nuclear membrane microtubule tethering complex"
}